{
  "term_id": "GO:0160040",
  "gene_name": "Uncharacterized protein C21orf62",
  "gene_symbol": "C21orf62",
  "term_label": "mitocytosis",
  "gene": "UniProtKB:Q9NYP8"
}